{
  "gene_name": "Eukaryotic translation initiation factor 2D",
  "gene": "UniProtKB:P41214",
  "term_id": "GO:0001731",
  "term_label": "formation of translation preinitiation complex",
  "gene_symbol": "EIF2D"
}